{
  "gene_symbol": "ERAL1",
  "gene": "UniProtKB:O75616",
  "term_label": "ribosomal small subunit binding",
  "term_id": "GO:0043024",
  "gene_name": "GTPase Era, mitochondrial"
}